{
  "term_id": "UNKNOWN:0003",
  "gene_symbol": "TMEM25",
  "gene": "UniProtKB:Q86YD3",
  "term_label": "Unknown cellular component",
  "gene_name": "Transmembrane protein 25"
}